{
  "term_label": "Unknown biological process",
  "gene": "UniProtKB:Q96L08",
  "term_id": "UNKNOWN:0002",
  "gene_name": "Sushi domain-containing protein 3",
  "gene_symbol": "SUSD3"
}